{
  "gene_name": "STAG3-like protein 3",
  "term_label": "Unknown cellular component",
  "gene": "UniProtKB:P0CL85",
  "term_id": "UNKNOWN:0003",
  "gene_symbol": "STAG3L3"
}